{
  "gene_name": "Latent-transforming growth factor beta-binding protein 4",
  "gene": "UniProtKB:Q8N2S1",
  "gene_symbol": "LTBP4",
  "term_id": "GO:0005615",
  "term_label": "extracellular space"
}